{
  "gene_symbol": "FAM20A",
  "gene_name": "Pseudokinase FAM20A",
  "term_label": "extracellular space",
  "gene": "UniProtKB:Q96MK3",
  "term_id": "GO:0005615"
}